{
  "gene": "UniProtKB:Q6ZNQ3",
  "gene_symbol": "LRRC69",
  "term_id": "UNKNOWN:0003",
  "term_label": "Unknown cellular component",
  "gene_name": "Leucine-rich repeat-containing protein 69"
}